{
  "gene": "UniProtKB:Q5JPH6",
  "term_id": "GO:0005739",
  "term_label": "mitochondrion",
  "gene_name": "Probable glutamate--tRNA ligase, mitochondrial",
  "gene_symbol": "EARS2"
}